L-fuculose-phosphate aldolase activity [GO:0008738] (molecular function) Relationships: is a type of aldehyde-lyase activity [GO:0016832] Also known as: L-fuculose 1-phosphate aldolase activity, L-fuculose-1-phosphate S-lactaldehyde-lyase (glycerone-phosphate-forming), L-fuculose-1-phosphate lactaldehyde-lyase activity, fuculose aldolase activity Definition: Catalysis of the reaction: L-fuculose 1-phosphate = (S)-lactaldehyde + glycerone phosphate. Sources: EC:4.1.2.17, RHEA:12933